{
  "gene_name": "DNL-type zinc finger protein",
  "gene": "UniProtKB:Q5SXM8",
  "gene_symbol": "DNLZ",
  "term_label": "protein folding",
  "term_id": "GO:0006457"
}